meiotic spindle pole [GO:0090619] (cellular component) Definition: Either of the ends of a meiotic spindle, a spindle that forms as part of meiosis, where spindle microtubules are organized; usually contains a microtubule organizing center and accessory molecules, spindle microtubules and astral microtubules. Relationships: is a type of spindle pole [GO:0000922]; is part of meiotic spindle [GO:0072687] References: PMID:18250200 Sources: GOC:ha